regulation of melanosome organization [GO:1903056] (biological process) Subtypes: negative regulation of melanosome organization [GO:1903057], positive regulation of melanosome organization [GO:1903058] Relationships: is a type of GO:0033043; regulates melanosome organization [GO:0032438] Also known as: regulation of melanosome organisation, regulation of melanosome organization and biogenesis Note: Lack of the transcription factor Zeb2 Q9R0G7 leads to spherical melanosomes with irregular borders, in contrast to the rod-shaped melanosomes of ZEB2MCWT hair follicles Definition: Any process that modulates the frequency, rate or extent of melanosome organization. References: PMID:24769727 Sources: GOC:BHF, GOC:TermGenie, GOC:rl, GO_REF:0000058